L-methionine catabolic process via 2-oxobutanoate [GO:0019458] (biological process) Also known as: methionine breakdown via 2-oxobutanoate, methionine degradation via 2-oxobutanoate Relationships: is_a L-methionine catabolic process [GO:0009087] Definition: The chemical reactions and pathways resulting in the breakdown of L-methionine, via the intermediate 2-oxobutanoate. Sources: GOC:go_curators